{
  "gene_name": "RWD domain-containing protein 2A",
  "term_label": "Unknown molecular function",
  "term_id": "UNKNOWN:0001",
  "gene_symbol": "RWDD2A",
  "gene": "UniProtKB:Q9UIY3"
}